opsonization [GO:0008228] (biological process) Relationships: is a type of immune effector process [GO:0002252]; positively regulates phagocytosis, recognition [GO:0006910] Regulation: regulated by regulation of opsonization [GO:1903027]; positively regulated by positive regulation of opsonization [GO:1903028] Definition: The process in which a microorganism (or other particulate material) is rendered more susceptible to phagocytosis by coating with an opsonin, a blood serum protein such as a complement component or antibody. Sources: GOC:add, GOC:mah, ISBN:0198506732, ISBN:068340007X, ISBN:0781735149